{
  "gene_name": "Phosphoenolpyruvate carboxykinase [GTP], mitochondrial",
  "gene_symbol": "PCK2",
  "gene": "UniProtKB:Q16822",
  "term_label": "gluconeogenesis",
  "term_id": "GO:0006094"
}